{
  "gene": "UniProtKB:Q9BYZ6",
  "gene_name": "Rho-related BTB domain-containing protein 2",
  "term_id": "GO:0005525",
  "term_label": "GTP binding",
  "gene_symbol": "RHOBTB2"
}